{
  "term_id": "GO:0034314",
  "gene": "UniProtKB:Q8TF30",
  "term_label": "Arp2/3 complex-mediated actin nucleation",
  "gene_symbol": "WHAMM",
  "gene_name": "WASP homolog-associated protein with actin, membranes and microtubules"
}